{
  "term_id": "GO:0007263",
  "gene_symbol": "NOS3",
  "gene": "UniProtKB:P29474",
  "gene_name": "Nitric oxide synthase 3",
  "term_label": "nitric oxide mediated signal transduction"
}